{
  "gene_symbol": "GALR1",
  "gene_name": "Galanin receptor type 1",
  "term_label": "neuropeptide signaling pathway",
  "gene": "UniProtKB:P47211",
  "term_id": "GO:0007218"
}